{
  "gene_name": "Homeobox protein TGIF1",
  "gene": "UniProtKB:Q15583",
  "term_label": "RNA polymerase II cis-regulatory region sequence-specific DNA binding",
  "gene_symbol": "TGIF1",
  "term_id": "GO:0000978"
}